{
  "term_id": "UNKNOWN:0001",
  "gene_name": "Protein FAM153B",
  "term_label": "Unknown molecular function",
  "gene": "UniProtKB:P0C7A2",
  "gene_symbol": "FAM153B"
}